{
  "term_label": "Unknown biological process",
  "gene": "UniProtKB:A6NIR3",
  "gene_symbol": "AGAP5",
  "gene_name": "Arf-GAP with GTPase, ANK repeat and PH domain-containing protein 5",
  "term_id": "UNKNOWN:0002"
}